{
  "term_id": "GO:0035914",
  "gene_symbol": "MYOD1",
  "term_label": "skeletal muscle cell differentiation",
  "gene": "UniProtKB:P15172",
  "gene_name": "Myoblast determination protein 1"
}